positive regulation of RNA export from nucleus [GO:0046833] (BP) Definition: Any process that activates or increases the frequency, rate or extent of directed movement of RNA from the nucleus into the cytoplasm. Sources: GOC:bf Also known as: positive regulation of RNA export from cell nucleus, positive regulation of RNA export out of nucleus, positive regulation of RNA transport from nucleus to cytoplasm, positive regulation of RNA-nucleus export, up regulation of RNA export from nucleus, up-regulation of RNA export from nucleus, upregulation of RNA export from nucleus, activation of RNA export from nucleus, stimulation of RNA export from nucleus Relationships: is a type of GO:0032241; is a type of GO:0046824; is a type of GO:0046831; positively regulates GO:0006405 Subtypes: positive regulation of tRNA export from nucleus [GO:2000240]